{
  "term_label": "cytoplasm",
  "gene_name": "Gametogenetin-binding protein 2",
  "term_id": "GO:0005737",
  "gene": "UniProtKB:Q9H3C7",
  "gene_symbol": "GGNBP2"
}